{
  "term_id": "GO:0047676",
  "gene_name": "Long-chain-fatty-acid--CoA ligase 6",
  "gene_symbol": "ACSL6",
  "gene": "UniProtKB:Q9UKU0",
  "term_label": "arachidonate-CoA ligase activity"
}